host cell endosome membrane [GO:0044175] (cellular component) Subtypes: host cell late endosome membrane [GO:0044185] Definition: The lipid bilayer surrounding a host cell endosome. Sources: GOC:jl Relationships: is a type of GO:0033644; is part of host cell endosome [GO:0044174] Also known as: host endosome membrane